{
  "gene": "UniProtKB:Q9NS82",
  "gene_symbol": "SLC7A10",
  "term_id": "UNKNOWN:0003",
  "term_label": "Unknown cellular component",
  "gene_name": "Asc-type amino acid transporter 1"
}